{
  "gene": "UniProtKB:Q07820",
  "gene_symbol": "MCL1",
  "term_id": "GO:0008053",
  "gene_name": "Induced myeloid leukemia cell differentiation protein Mcl-1",
  "term_label": "mitochondrial fusion"
}